2,5-dioxovalerate dehydrogenase (NADP+) activity [GO:0047533] (molecular function) Sources: EC:1.2.1.26, MetaCyc:25-DIOXOVALERATE-DEHYDROGENASE-RXN Definition: Catalysis of the reaction: 2,5-dioxopentanoate + NADP+ + H2O = 2-oxoglutarate + NADPH + H+. Relationships: is_a oxidoreductase activity, acting on the aldehyde or oxo group of donors, NAD or NADP as acceptor [GO:0016620] Also known as: 2,5-dioxopentanoate:NADP+ 5-oxidoreductase activity, 2-oxoglutarate semialdehyde dehydrogenase activity, alpha-ketoglutaric semialdehyde dehydrogenase activity